{
  "term_label": "Unknown biological process",
  "gene": "UniProtKB:Q58G82",
  "gene_symbol": "SYT14P1",
  "term_id": "UNKNOWN:0002",
  "gene_name": "Putative synaptotagmin-14-like protein"
}